{
  "gene_symbol": "GJB1",
  "gene_name": "Gap junction beta-1 protein",
  "gene": "UniProtKB:P08034",
  "term_id": "GO:0005243",
  "term_label": "gap junction channel activity"
}